{
  "gene_symbol": "CPO",
  "term_id": "GO:0005615",
  "gene_name": "Carboxypeptidase O",
  "term_label": "extracellular space",
  "gene": "UniProtKB:Q8IVL8"
}